DNA clamp unloader activity [GO:0061860] (molecular function) Definition: Facilitating the opening of the ring structure of the PCNA complex, or any of the related sliding clamp complexes, and their removal from the DNA duplex, driven by ATP hydrolysis. Also known as: DNA clamp unloading activity Relationships: is a type of GO:0008094; has part GO:0003677 References: PMID:23499004 Sources: GOC:vw